{
  "gene_symbol": "ATG7",
  "gene": "UniProtKB:O95352",
  "term_label": "cytoplasm",
  "gene_name": "Ubiquitin-like modifier-activating enzyme ATG7",
  "term_id": "GO:0005737"
}